{
  "gene_symbol": "UBE2D4",
  "gene": "UniProtKB:Q9Y2X8",
  "gene_name": "Ubiquitin-conjugating enzyme E2 D4",
  "term_label": "protein K48-linked ubiquitination",
  "term_id": "GO:0070936"
}